{
  "gene_name": "Kelch-like protein 3",
  "gene_symbol": "KLHL3",
  "term_id": "GO:0031463",
  "term_label": "Cul3-RING ubiquitin ligase complex",
  "gene": "UniProtKB:Q9UH77"
}